{
  "gene": "UniProtKB:Q9ULX5",
  "term_label": "endoplasmic reticulum organization",
  "term_id": "GO:0007029",
  "gene_name": "RING finger protein 112",
  "gene_symbol": "RNF112"
}